{
  "gene_name": "Myomegalin",
  "term_id": "GO:0005794",
  "gene": "UniProtKB:Q5VU43",
  "term_label": "Golgi apparatus",
  "gene_symbol": "PDE4DIP"
}